protein serine kinase activity [GO:0106310] (molecular function) Also known as: protein-serine kinase activity Definition: Catalysis of the reactions: ATP + protein serine = ADP + protein serine phosphate. Subtypes: [isocitrate dehydrogenase (NADP+)] kinase activity [GO:0008772] Relationships: is a type of protein kinase activity [GO:0004672] Note: Note that this term is to annotate proteins the specifically phosphorylate a serine residue on a protein. An example is human PIKFYVE (UniProt:Q9Y2I7). For dual specificity protein kinases, use 'protein serine/threonine kinase activity' ; GO:0004712. Sources: RHEA:17989